{
  "gene_symbol": "HLA-F",
  "term_label": "external side of plasma membrane",
  "gene_name": "HLA class I histocompatibility antigen, alpha chain F",
  "term_id": "GO:0009897",
  "gene": "UniProtKB:P30511"
}